{
  "term_label": "L-valine biosynthetic process",
  "term_id": "GO:0009099",
  "gene": "UniProtKB:A1L0T0",
  "gene_name": "2-hydroxyacyl-CoA lyase 2",
  "gene_symbol": "ILVBL"
}